{
  "gene_symbol": "ZDHHC23",
  "term_label": "protein-cysteine S-palmitoyltransferase activity",
  "gene": "UniProtKB:Q8IYP9",
  "term_id": "GO:0019706",
  "gene_name": "Palmitoyltransferase ZDHHC23"
}